{
  "gene": "UniProtKB:P56962",
  "gene_symbol": "STX17",
  "term_label": "intracellular protein transport",
  "term_id": "GO:0006886",
  "gene_name": "Syntaxin-17"
}